{
  "term_label": "Unknown biological process",
  "gene": "UniProtKB:A0A0A0MT97",
  "gene_symbol": "TRGJP1",
  "gene_name": "T cell receptor gamma joining P1 (Fragment)",
  "term_id": "UNKNOWN:0002"
}